{
  "gene": "UniProtKB:Q6UX72",
  "gene_symbol": "B3GNT9",
  "term_label": "UDP-glycosyltransferase activity",
  "term_id": "GO:0008194",
  "gene_name": "UDP-GlcNAc:betaGal beta-1,3-N-acetylglucosaminyltransferase 9"
}